{
  "gene_name": "Protein STPG3",
  "gene_symbol": "STPG3",
  "term_id": "UNKNOWN:0001",
  "gene": "UniProtKB:Q8N7X2",
  "term_label": "Unknown molecular function"
}